dimethyl sulfoxide metabolic process [GO:0018907] (biological process) Also known as: DMSO metabolic process, DMSO metabolism, dimethyl sulfoxide metabolism, dimethyl sulphoxide metabolic process, dimethyl sulphoxide metabolism Sources: GOC:curators Definition: The chemical reactions and pathways involving dimethyl sulfoxide, DMSO (C2H6OS), an alkyl sulfoxide that is practically odorless in its purified form. As a highly polar organic liquid, it is a powerful solvent. Its biological activities include the ability to penetrate plant and animal tissues and to preserve living cells during freezing. Relationships: is a type of sulfur compound metabolic process [GO:0006790]